{
  "term_id": "GO:0006281",
  "term_label": "DNA repair",
  "gene_name": "ATR-interacting protein",
  "gene_symbol": "ATRIP",
  "gene": "UniProtKB:Q8WXE1"
}